{
  "term_id": "GO:0048786",
  "gene": "UniProtKB:O75335",
  "term_label": "presynaptic active zone",
  "gene_name": "Liprin-alpha-4",
  "gene_symbol": "PPFIA4"
}